{
  "gene_name": "Protein cordon-bleu",
  "term_label": "dendritic growth cone",
  "gene_symbol": "COBL",
  "gene": "UniProtKB:O75128",
  "term_id": "GO:0044294"
}